{
  "term_id": "UNKNOWN:0003",
  "gene_name": "Thiamin pyrophosphokinase 1",
  "gene_symbol": "TPK1",
  "term_label": "Unknown cellular component",
  "gene": "UniProtKB:Q9H3S4"
}